{
  "gene_symbol": "FNIP2",
  "term_id": "GO:0042030",
  "gene_name": "Folliculin-interacting protein 2",
  "term_label": "ATPase inhibitor activity",
  "gene": "UniProtKB:Q9P278"
}